DNA double-strand break attachment to nuclear envelope [GO:1990683] (biological process) References: PMID:24943839 Relationships: is a type of chromosome attachment to the nuclear envelope [GO:0097240] Definition: A process in which the DNA double-strand breaks are attached to the inner surface of the nuclear envelope proximal to the spindle pole body, or iMTOCs.